{
  "gene": "UniProtKB:Q9GZV9",
  "term_id": "GO:0008083",
  "gene_name": "Fibroblast growth factor 23",
  "term_label": "growth factor activity",
  "gene_symbol": "FGF23"
}